{
  "term_id": "GO:0006357",
  "gene_name": "Zinc finger protein 75A",
  "term_label": "regulation of transcription by RNA polymerase II",
  "gene_symbol": "ZNF75A",
  "gene": "UniProtKB:Q96N20"
}